anterior head development [GO:0097065] (biological process) Relationships: is a type of head development [GO:0060322] References: PMID:14695376, PMID:15857913 Sources: GOC:yaf Definition: The process whose specific outcome is the progression of the anterior part of the head over time, from its formation to the mature structure. Regulation: regulated by regulation of anterior head development [GO:2000742]; negatively regulated by GO:2000743; positively regulated by positive regulation of anterior head development [GO:2000744]